{
  "gene": "UniProtKB:O60296",
  "term_label": "dendrite",
  "gene_symbol": "TRAK2",
  "term_id": "GO:0030425",
  "gene_name": "Trafficking kinesin-binding protein 2"
}